{
  "term_id": "UNKNOWN:0003",
  "term_label": "Unknown cellular component",
  "gene_name": "T-complex protein 11-like protein 1",
  "gene_symbol": "TCP11L1",
  "gene": "UniProtKB:Q9NUJ3"
}